lipid kinase activity [GO:0001727] (molecular function) Regulation: regulated by regulation of lipid kinase activity [GO:0043550]; positively regulated by positive regulation of lipid kinase activity [GO:0090218] Sources: GOC:hjd Relationships: is_a kinase activity [GO:0016301] Definition: Catalysis of the phosphorylation of a simple or complex lipid. Subtypes: GO:0001729, ATP-dependent diacylglycerol kinase activity [GO:0004143], sphingosine kinase activity [GO:0008481], phosphatidylinositol kinase activity [GO:0052742], CTP-dependent diacylglycerol kinase activity [GO:0141035]